MSL complex [GO:0072487] (cellular component) Definition: A histone acetyltransferase complex that catalyzes the acetylation of a histone H4 lysine residue at position 16. In human, it contains the catalytic subunit MOF, and MSL1, MSL2 and MSL3. Relationships: is a type of H4 histone acetyltransferase complex [GO:1902562] References: PMID:16227571, PMID:20018852